leukotriene-C4 synthase activity [GO:0004464] (molecular function) Note: Note that this function was EC:2.5.1.37. Sources: EC:4.4.1.20, RHEA:17617 Relationships: is a type of GO:0016846 Definition: Catalysis of the reaction: leukotriene C(4) = glutathione + leukotriene A(4). Also known as: (7E,9E,11Z,14Z)-(5S,6R)-5,6-epoxyicosa-7,9,11,14-tetraenoate:glutathione leukotriene-transferase (epoxide-ring-opening), (7E,9E,11Z,14Z)-(5S,6R)-6-(glutathion-S-yl)-5-hydroxyicosa-7,9,11,14-tetraenoate glutathione-lyase (epoxide-forming), LTC(4) synthase activity, LTC(4) synthetase activity, LTC4 synthase activity, LTC4 synthetase activity, leukotriene A(4):glutathione S-leukotrienyltransferase activity, leukotriene A4:glutathione S-leukotrienyltransferase activity, leukotriene C(4) synthetase activity, leukotriene C4 synthetase activity, leukotriene-C4 glutathione-lyase (leukotriene-A4-forming)